negative regulation of response to acetate [GO:1901458] (biological process) Also known as: down regulation of response to acetate, down-regulation of response to acetate, downregulation of response to acetate, inhibition of response to acetate Relationships: is a type of negative regulation of response to stimulus [GO:0048585]; is a type of regulation of response to acetate [GO:1901457]; negatively regulates response to acetate [GO:0010034] Definition: Any process that stops, prevents or reduces the frequency, rate or extent of response to acetate. Sources: GOC:TermGenie, GOC:mengo_curators